{
  "term_label": "glucuronosyl-N-acetylgalactosaminyl-proteoglycan 4-beta-N-acetylgalactosaminyltransferase activity",
  "term_id": "GO:0047238",
  "gene_symbol": "CSGALNACT2",
  "gene": "UniProtKB:Q8N6G5",
  "gene_name": "Chondroitin sulfate N-acetylgalactosaminyltransferase 2"
}